{
  "gene_symbol": "ABCD4",
  "gene": "UniProtKB:O14678",
  "gene_name": "Lysosomal cobalamin transporter ABCD4",
  "term_id": "GO:0042760",
  "term_label": "very long-chain fatty acid catabolic process"
}